{
  "term_id": "GO:0035249",
  "gene": "UniProtKB:O15399",
  "gene_symbol": "GRIN2D",
  "term_label": "synaptic transmission, glutamatergic",
  "gene_name": "Glutamate receptor ionotropic, NMDA 2D"
}